positive regulation of amoeboid sperm motility [GO:1905418] (biological process) Definition: Any process that activates or increases the frequency, rate or extent of amoeboid sperm motility. Sources: GOC:TermGenie, GOC:cilia, GOC:krc, GO_REF:0000058 Also known as: positive regulation of ameboid sperm motility, positive regulation of ameboid sperm movement, positive regulation of amoeboid sperm movement, up regulation of ameboid sperm motility, up regulation of ameboid sperm movement, up regulation of amoeboid sperm motility, up regulation of amoeboid sperm movement, up-regulation of ameboid sperm motility, up-regulation of ameboid sperm movement, up-regulation of amoeboid sperm motility, up-regulation of amoeboid sperm movement, upregulation of ameboid sperm motility, upregulation of ameboid sperm movement, upregulation of amoeboid sperm motility, upregulation of amoeboid sperm movement, activation of ameboid sperm motility, activation of ameboid sperm movement, activation of amoeboid sperm motility, activation of amoeboid sperm movement Relationships: is a type of regulation of amoeboid sperm motility [GO:1905416]; is a type of GO:2000147; is a type of positive regulation of reproductive process [GO:2000243]; positively regulates amoeboid sperm motility [GO:0097723]